{
  "gene": "UniProtKB:O60548",
  "gene_symbol": "FOXD2",
  "gene_name": "Forkhead box protein D2",
  "term_id": "GO:0000981",
  "term_label": "DNA-binding transcription factor activity, RNA polymerase II-specific"
}